{
  "gene_name": "Kallikrein-14",
  "gene_symbol": "KLK14",
  "gene": "UniProtKB:Q9P0G3",
  "term_label": "extracellular space",
  "term_id": "GO:0005615"
}